{
  "gene": "UniProtKB:Q86SJ2",
  "gene_symbol": "AMIGO2",
  "term_id": "UNKNOWN:0001",
  "gene_name": "Amphoterin-induced protein 2",
  "term_label": "Unknown molecular function"
}